{
  "gene": "UniProtKB:P47992",
  "gene_symbol": "XCL1",
  "gene_name": "Lymphotactin",
  "term_id": "GO:0005615",
  "term_label": "extracellular space"
}